beta-catenin destruction complex binding [GO:1904713] (molecular function) Also known as: APC-Axin-1-beta-catenin complex binding, Axin-APC-beta-catenin-GSK3B complex binding, BDC binding, beta-catenin degradation complex binding, 23S APC complex binding Relationships: is a type of protein-containing complex binding [GO:0044877] Definition: Binding to a beta-catenin destruction complex. References: PMID:22899650 Sources: GOC:PARL, GOC:TermGenie, GOC:bf